indole phytoalexin biosynthetic process [GO:0009700] (biological process) Relationships: is a type of indole-containing compound biosynthetic process [GO:0042435]; is a type of phytoalexin biosynthetic process [GO:0052315] Sources: GOC:sm, ISBN:0198547684 Subtypes: GO:0010120 Definition: The chemical reactions and pathways resulting in the formation of indole phytoalexins, any indole compound produced by plants as part of their defense response. Also known as: indole phytoalexin anabolism, indole phytoalexin biosynthesis, indole phytoalexin formation, indole phytoalexin synthesis